{
  "gene_symbol": "TLR4",
  "term_id": "GO:0005886",
  "gene": "UniProtKB:O00206",
  "gene_name": "Toll-like receptor 4",
  "term_label": "plasma membrane"
}